{
  "gene_name": "Sodium channel protein type 3 subunit alpha",
  "gene_symbol": "SCN3A",
  "term_id": "GO:0001518",
  "term_label": "voltage-gated sodium channel complex",
  "gene": "UniProtKB:Q9NY46"
}